{
  "gene_symbol": "TMEM214",
  "term_label": "Unknown biological process",
  "term_id": "UNKNOWN:0002",
  "gene": "UniProtKB:Q6NUQ4",
  "gene_name": "Transmembrane protein 214"
}